{
  "gene_symbol": "UBE2O",
  "gene": "UniProtKB:Q9C0C9",
  "gene_name": "(E3-independent) E2 ubiquitin-conjugating enzyme",
  "term_label": "ubiquitin conjugating enzyme activity",
  "term_id": "GO:0061631"
}